{
  "gene_symbol": "PDGFC",
  "term_label": "positive regulation of cell migration",
  "term_id": "GO:0030335",
  "gene_name": "Platelet-derived growth factor C",
  "gene": "UniProtKB:Q9NRA1"
}